filopodium assembly [GO:0046847] (biological process) Regulation: RO_0002211 by regulation of filopodium assembly [GO:0051489]; RO_0002212 by negative regulation of filopodium assembly [GO:0051490]; RO_0002213 by positive regulation of filopodium assembly [GO:0051491] Subtypes: endothelial tip cell filopodium assembly [GO:0120084] Definition: The assembly of a filopodium, a thin, stiff protrusion extended by the leading edge of a motile cell such as a crawling fibroblast or amoeba, or an axonal growth cone. Also known as: filopodia biosynthesis, filopodia formation, filopodium formation Relationships: is a type of plasma membrane bounded cell projection assembly [GO:0120031] References: PMID:16337369, PMID:18464790 Sources: GOC:dph, GOC:mah, GOC:tb